annuli extracellular matrix [GO:0060107] (cellular component) Relationships: is a type of cellular anatomical structure [GO:0110165]; is part of cortical layer of collagen and cuticulin-based cuticle extracellular matrix [GO:0060106] Definition: The extracellular matrix that is a regularly spaced circumferential ridge present in the cortical region of the cuticle. Annuli are delineated by annular furrows and are present throughout the cuticle with the exception of lateral regions where longitudinal alae are present. Sources: GOC:dph, GOC:kmv, ISSN:15518507 Also known as: annulae, annular rings, annule(s), annulus